{
  "term_id": "GO:0000226",
  "term_label": "microtubule cytoskeleton organization",
  "gene": "UniProtKB:Q9BUY7",
  "gene_name": "EF-hand calcium-binding domain-containing protein 11",
  "gene_symbol": "EFCAB11"
}